meristem maintenance [GO:0010073] (biological process) Definition: Any process involved in maintaining the identity, size and shape of a meristem. Sources: GOC:tb Relationships: is a type of multicellular organismal process [GO:0032501]; is part of meristem development [GO:0048507]